dAMP kinase activity [GO:0047506] (molecular function) Also known as: (deoxy)adenylate kinase activity, ATP:(d)AMP phosphotransferase activity Sources: RHEA:23100 Relationships: is a type of deoxynucleoside phosphate kinase activity, ATP as phosphate donor [GO:0047507] Definition: Catalysis of the reaction: dAMP + ATP = dADP + ADP.